{
  "term_id": "GO:0050911",
  "gene": "UniProtKB:Q8N349",
  "gene_symbol": "OR2L13",
  "gene_name": "Olfactory receptor 2L13",
  "term_label": "detection of chemical stimulus involved in sensory perception of smell"
}